DNA-directed RNA polymerase activity [GO:0003899] (molecular function) Sources: EC:2.7.7.6 Definition: Catalysis of the reaction: nucleoside triphosphate + RNA(n) = diphosphate + RNA(n+1). Utilizes a DNA template, i.e. the catalysis of DNA-template-directed extension of the 3'-end of an RNA strand by one nucleotide at a time. Can initiate a chain 'de novo'. Relationships: is a type of GO:0034062; is part of RNA biosynthetic process [GO:0032774] Also known as: transcriptase, DNA-directed RNA polymerase I activity, DNA-directed RNA polymerase II activity, DNA-directed RNA polymerase III activity, RNA polymerase I activity, RNA polymerase II activity, RNA polymerase III activity, RNA polymerase IV activity, RNA polymerase V activity, C RNA formation factors, C ribonucleic acid formation factors, DNA-dependent RNA nucleotidyltransferase activity, DNA-dependent RNA polymerase activity, DNA-dependent ribonucleate nucleotidyltransferase activity, RNA nucleotidyltransferase (DNA-directed) activity, deoxyribonucleic acid-dependent ribonucleic acid polymerase activity, nucleoside-triphosphate:RNA nucleotidyltransferase (DNA-directed) activity